{
  "gene": "UniProtKB:P05160",
  "gene_name": "Coagulation factor XIII B chain",
  "term_id": "UNKNOWN:0001",
  "gene_symbol": "F13B",
  "term_label": "Unknown molecular function"
}